{
  "term_id": "UNKNOWN:0003",
  "gene": "UniProtKB:Q9Y2K5",
  "gene_name": "R3H domain-containing protein 2",
  "term_label": "Unknown cellular component",
  "gene_symbol": "R3HDM2"
}